{
  "gene_name": "Disintegrin and metalloproteinase domain-containing protein 12",
  "term_id": "GO:0006508",
  "term_label": "proteolysis",
  "gene_symbol": "ADAM12",
  "gene": "UniProtKB:O43184"
}